{
  "term_label": "Unknown cellular component",
  "gene": "UniProtKB:Q02386",
  "term_id": "UNKNOWN:0003",
  "gene_name": "Zinc finger protein 45",
  "gene_symbol": "ZNF45"
}